{
  "term_label": "RNA polymerase II cis-regulatory region sequence-specific DNA binding",
  "term_id": "GO:0000978",
  "gene": "UniProtKB:Q12951",
  "gene_symbol": "FOXI1",
  "gene_name": "Forkhead box protein I1"
}